{
  "gene_name": "Putative uncharacterized protein encoded by MAPKAPK5-AS1",
  "gene_symbol": "MAPKAPK5-AS1",
  "term_id": "UNKNOWN:0003",
  "gene": "UniProtKB:Q8N8E1",
  "term_label": "Unknown cellular component"
}